{
  "gene": "UniProtKB:Q6XPR3",
  "gene_name": "Repetin",
  "term_id": "GO:0001533",
  "term_label": "cornified envelope",
  "gene_symbol": "RPTN"
}